{
  "term_label": "cell-cell adhesion mediator activity",
  "gene": "UniProtKB:Q9BQT9",
  "term_id": "GO:0098632",
  "gene_symbol": "CLSTN3",
  "gene_name": "Calsyntenin-3"
}